{
  "term_id": "GO:0034237",
  "term_label": "protein kinase A regulatory subunit binding",
  "gene_name": "Actin-binding protein WASF1",
  "gene": "UniProtKB:Q92558",
  "gene_symbol": "WASF1"
}